{
  "gene_symbol": "CLDN7",
  "term_label": "Unknown molecular function",
  "gene_name": "Claudin-7",
  "term_id": "UNKNOWN:0001",
  "gene": "UniProtKB:O95471"
}